{
  "gene_name": "Transient receptor potential cation channel subfamily M member 6",
  "gene_symbol": "TRPM6",
  "term_label": "calcium ion transport",
  "gene": "UniProtKB:Q9BX84",
  "term_id": "GO:0006816"
}